{
  "term_label": "Unknown molecular function",
  "gene_symbol": "PRR16",
  "gene": "UniProtKB:Q569H4",
  "gene_name": "Protein Largen",
  "term_id": "UNKNOWN:0001"
}